{
  "gene_name": "Bromodomain adjacent to zinc finger domain protein 1A",
  "term_label": "regulation of heterochromatin formation",
  "gene_symbol": "BAZ1A",
  "term_id": "GO:0031445",
  "gene": "UniProtKB:Q9NRL2"
}